{
  "term_label": "vesicle fusion",
  "gene": "UniProtKB:Q13277",
  "gene_name": "Syntaxin-3",
  "gene_symbol": "STX3",
  "term_id": "GO:0006906"
}